{
  "gene_name": "Sperm-associated antigen 16 protein",
  "term_label": "axonemal central apparatus",
  "gene_symbol": "SPAG16",
  "term_id": "GO:1990716",
  "gene": "UniProtKB:Q8N0X2"
}